{
  "gene_name": "ELAV-like protein 4",
  "term_id": "UNKNOWN:0003",
  "gene_symbol": "ELAVL4",
  "gene": "UniProtKB:P26378",
  "term_label": "Unknown cellular component"
}